{
  "gene_symbol": "BAZ2A",
  "term_label": "Unknown molecular function",
  "term_id": "UNKNOWN:0001",
  "gene": "UniProtKB:Q9UIF9",
  "gene_name": "Bromodomain adjacent to zinc finger domain protein 2A"
}